{
  "gene_name": "Cytochrome P450 2A7",
  "term_id": "GO:0019373",
  "gene_symbol": "CYP2A7",
  "gene": "UniProtKB:P20853",
  "term_label": "epoxygenase P450 pathway"
}